synaptic vesicle clustering [GO:0097091] (biological process) Relationships: is_a GO:0097479; is part of synaptic vesicle cycle [GO:0099504] References: PMID:19900895, PMID:7568108 Sources: GOC:ans, GOC:pr Regulation: regulated by regulation of synaptic vesicle clustering [GO:2000807]; negatively regulated by negative regulation of synaptic vesicle clustering [GO:2000808]; positively regulated by positive regulation of synaptic vesicle clustering [GO:2000809] Definition: The process that results in grouping synaptic vesicles in presynaptic structures.